{
  "gene_name": "Homeobox protein DLX-5",
  "term_id": "GO:0048706",
  "term_label": "embryonic skeletal system development",
  "gene": "UniProtKB:P56178",
  "gene_symbol": "DLX5"
}